female pronucleus assembly [GO:0035038] (biological process) Definition: Assembly of the haploid nucleus of the unfertilized egg. Sources: GOC:bf, ISBN:0582227089 Relationships: is a type of nucleus organization [GO:0006997]; is a type of organelle assembly [GO:0070925]; is part of single fertilization [GO:0007338]